{
  "gene_symbol": "TMEM198",
  "term_label": "plasma membrane",
  "term_id": "GO:0005886",
  "gene": "UniProtKB:Q66K66",
  "gene_name": "Transmembrane protein 198"
}